{
  "term_label": "channel activity",
  "term_id": "GO:0015267",
  "gene_symbol": "BCL2L10",
  "gene": "UniProtKB:Q9HD36",
  "gene_name": "Bcl-2-like protein 10"
}